PRC1 complex binding [GO:0140259] (MF) References: PMID:15280237 Relationships: is a type of protein-containing complex binding [GO:0044877] Definition: Binding to a PRC1 complex.